Golgi transport vesicle coating [GO:0048200] (biological process) Definition: The addition of specific coat proteins to Golgi membranes during the formation of transport vesicles. References: PMID:10219233 Sources: GOC:jid, GOC:mah, ISBN:0716731363 Subtypes: GO:0048202, COPI coating of Golgi vesicle [GO:0048205] Relationships: is a type of vesicle coating [GO:0006901]; is part of GO:0048194; is part of GO:0048199 Also known as: dictyosome transport vesicle coating